type 3 somatostatin receptor binding [GO:0031880] (molecular function) Relationships: is a type of GO:0031877 Definition: Binding to a type 3 somatostatin receptor. Also known as: type 3 somatostatin receptor ligand Sources: GOC:mah, GOC:nln